catalytic complex [GO:1902494] (cellular component) Definition: A protein complex which is capable of catalytic activity. Subtypes: phosphopyruvate hydratase complex [GO:0000015], histone deacetylase complex [GO:0000118], GO:0005601, GO:0005697, fatty acid synthase complex [GO:0005835], GO:0005839, anthranilate synthase complex [GO:0005950], carbamoyl-phosphate synthase complex [GO:0005951], calcium- and calmodulin-dependent protein kinase complex [GO:0005954], guanylate cyclase complex, soluble [GO:0008074], 1-alkyl-2-acetylglycerophosphocholine esterase complex [GO:0008247], 3-isopropylmalate dehydratase complex [GO:0009316], acetyl-CoA carboxylase complex [GO:0009317], exodeoxyribonuclease VII complex [GO:0009318], GO:0009320, phenylalanine-tRNA ligase complex [GO:0009328], DNA topoisomerase type II (double strand cut, ATP-hydrolyzing) complex [GO:0009330], GO:0009332, sulfite reductase complex (NADPH) [GO:0009337], exodeoxyribonuclease V complex [GO:0009338], beta-galactosidase complex [GO:0009341], GO:0009344, GO:0009345, ATP-independent citrate lyase complex [GO:0009346], ethanolamine ammonia-lyase complex [GO:0009350], aminodeoxychorismate synthase complex [GO:0009356], enterobactin synthetase complex [GO:0009366], endopeptidase Clp complex [GO:0009368], magnesium chelatase complex [GO:0010007], thioglucosidase complex [GO:0010169], pyrophosphate-dependent phosphofructokinase complex [GO:0010316], pyrophosphate-dependent phosphofructokinase complex, alpha-subunit complex [GO:0010317], pyrophosphate-dependent phosphofructokinase complex, beta-subunit complex [GO:0010318], GO:0010598, aminoacyl-tRNA synthetase multienzyme complex [GO:0017101], GO:0017109, phosphoenolpyruvate-dependent sugar phosphotransferase complex [GO:0019197], dynein complex [GO:0030286], GO:0030877, ADPG pyrophosphorylase complex [GO:0030929], glutamyl-tRNA(Gln) amidotransferase complex [GO:0030956], GO:0031250, Elg1 RFC-like complex [GO:0031391], invertasome [GO:0031421], box H/ACA snoRNP complex [GO:0031429], SUMO activating enzyme complex [GO:0031510], ribonuclease H2 complex [GO:0032299], DNA helicase complex [GO:0033202], elongator holoenzyme complex [GO:0033588], GO:0034081, GCH1 complex [GO:0034615], urease complex [GO:0035550], glutathione synthase complex [GO:0036087], GO:0043033, [Ni-Fe] hydrogenase complex [GO:0044569], acetyl-CoA decarbonylase/synthase-carbon monoxide dehydrogenase complex [GO:0044672], 7,8-didemethyl-8-hydroxy-5-deazariboflavin synthase complex [GO:0044673], formyl-methanofuran dehydrogenase (tungsten enzyme) complex [GO:0044675], GO:0044676, methyl-tetrahydromethanopterin:coenzyme M methyltransferase complex [GO:0044677], sulfopyruvate decarboxylase complex [GO:0044681], tricarboxylic acid cycle heteromeric enzyme complex [GO:0045239], GO:0045259, GO:0045283, mRNA editing complex [GO:0045293], GO:0048492, tRNA-specific adenosine-34 deaminase complex [GO:0052718], GO:0061576, cytochrome complex [GO:0070069], GO:0070214, CD20-Lck-Fyn complex [GO:0070331], CD20-Lck-Lyn-Fyn complex [GO:0070332], DNA ligase III-XRCC1 complex [GO:0070421], lysosomal multienzyme complex [GO:0070559], GO:0070765, catalytic step 1 spliceosome [GO:0071012], GO:0071013, alphav-beta3 integrin-ADAM15 complex [GO:0071057], alphav-beta3 integrin-ADAM23 complex [GO:0071067], fibronectin-tissue transglutaminase complex [GO:0071078], alpha5-beta1 integrin-tissue transglutaminase complex [GO:0071088], alphaV-beta3 integrin-tissue transglutaminase complex [GO:0071089], alphaIIb-beta3 integrin-fibronectin-tissue transglutaminase complex [GO:0071090], alpha1-beta1 integrin-tissue transglutaminase complex [GO:0071091], alpha3-beta1 integrin-tissue transglutaminase complex [GO:0071092], alpha5-beta1 integrin-fibronectin-tissue transglutaminase complex [GO:0071093], phosphopantothenoylcysteine decarboxylase complex [GO:0071513], box H/ACA scaRNP complex [GO:0072589], tRNA-splicing ligase complex [GO:0072669], ripoptosome [GO:0097342], viral terminase, large subunit [GO:0098009], GO:0106055, hydroxyisourate hydrolase complex [GO:0106232], ubiquinone biosynthesis complex [GO:0110142], ubiquitin activating enzyme complex [GO:0120123], GO:0120500, serine-tRNA ligase complex [GO:0140715], GO:0170010, 2-iminoacetate synthase complex [GO:1902508], glucosidase complex [GO:1902687], glutamate decarboxylase complex [GO:1902793], ornithine carbamoyltransferase inhibitor complex [GO:1903269], phosphatase complex [GO:1903293], GO:1903600, carbon phosphorus lyase complex [GO:1904176], ATPase complex [GO:1904949], heparanase complex [GO:1904974], methylcrotonoyl-CoA carboxylase complex [GO:1905202], endonuclease complex [GO:1905348], exoribonuclease complex [GO:1905354], GTPase complex [GO:1905360], GO:1905368, beta-N-acetylhexosaminidase complex [GO:1905379], GO:1990143, oxidoreductase complex [GO:1990204], intramolecular phosphotransferase complex [GO:1990233], GO:1990234, xylanosome [GO:1990358], GO:1990391 Relationships: is a type of protein-containing complex [GO:0032991] References: PMID:8077207 Sources: GOC:TermGenie, GOC:bhm Also known as: enzyme complex